antennal joint development [GO:0048098] (biological process) Sources: GOC:jid Definition: The process whose specific outcome is the progression of the antennal joint over time, from its formation to the mature structure. The antennal joint is the joint between antennal segments. Relationships: is a type of GO:0048856; is part of antennal development [GO:0007469]